type I pilus assembly [GO:0140623] (biological process) Also known as: T1P assembly, type 1 pilus biogenesis, type I fimbria assembly, type I fimbria biogenesis, type I fimbriae assembly, type I fimbriae biogenesis, type I fimbrial assembly, type I fimbrial biogenesis, type I fimbrium assembly, type I fimbrium biogenesis Relationships: is a type of pilus assembly [GO:0009297] Definition: The assembly from its constituent parts of a type I pilus. References: PMID:1679330